{
  "term_id": "GO:0005762",
  "gene_symbol": "MRPL47",
  "gene_name": "Large ribosomal subunit protein uL29m",
  "term_label": "mitochondrial large ribosomal subunit",
  "gene": "UniProtKB:Q9HD33"
}